succinate-hydroxymethylglutarate CoA-transferase activity [GO:0047369] (molecular function) Definition: Catalysis of the reaction: (S)-3-hydroxy-3-methylglutarate + succinyl-CoA = 3-hydroxy-3-methyl-glutaryl-CoA + succinate. Sources: EC:2.8.3.13, MetaCyc:2.8.3.13-RXN Also known as: dicarboxyl-CoA:dicarboxylic acid coenzyme A transferase activity, hydroxymethylglutarate coenzyme A-transferase activity, succinate:(S)-3-hydroxy-3-methylglutarate CoA-transferase activity Relationships: is a type of CoA-transferase activity [GO:0008410]